{
  "gene_name": "Class E basic helix-loop-helix protein 41",
  "gene": "UniProtKB:Q9C0J9",
  "term_id": "GO:0000122",
  "term_label": "negative regulation of transcription by RNA polymerase II",
  "gene_symbol": "BHLHE41"
}